negative regulation of mitochondrial membrane permeability [GO:0035795] (biological process) Subtypes: negative regulation of mitochondrial outer membrane permeabilization involved in apoptotic signaling pathway [GO:1901029], GO:1902109 Also known as: negative regulation of transport across mitochondrial membrane, mitochondrial membrane impermeabilization, mitochondrial membrane impermeability Definition: Any process that decreases the frequency, rate or extent of the passage or uptake of molecules by the mitochondrial membrane. References: PMID:10781072 Relationships: is_a regulation of mitochondrial membrane permeability [GO:0046902]; is a type of negative regulation of membrane permeability [GO:1905709]